pupal chitin-based cuticle development [GO:0008364] (biological process) Also known as: pupal cuticle anabolism, pupal cuticle formation, pupal cuticle synthesis Sources: GOC:bf, GOC:mtg_sensu, ISBN:0879694238 Definition: Synthesis and deposition of a chitin-based pupal cuticle. At the end of the prepupal period the insect is covered by the pupal cuticle which continues to be elaborated into the pupal period. An example of this is found in Drosophila melanogaster. Relationships: is a type of cuticle development involved in chitin-based cuticle molting cycle [GO:0042337]; is part of pupal development [GO:0035209]